{
  "term_label": "Golgi organization",
  "gene_symbol": "GORASP2",
  "gene": "UniProtKB:Q9H8Y8",
  "gene_name": "Golgi reassembly-stacking protein 2",
  "term_id": "GO:0007030"
}